{
  "gene_symbol": "FAM237A",
  "term_label": "Unknown biological process",
  "term_id": "UNKNOWN:0002",
  "gene_name": "Protein FAM237A",
  "gene": "UniProtKB:A0A1B0GTK4"
}